positive regulation of red or far-red light signaling pathway [GO:0090228] (BP) Sources: GOC:tb Also known as: positive regulation of phytochrome signaling pathway, positive regulation of red or far-red light signalling pathway Definition: Any process that increases the rate, frequency or extent of the red or far-red signaling pathway, the series of molecular signals initiated upon sensing by photoreceptor molecules of red light or far red light. Relationships: is a type of positive regulation of signal transduction [GO:0009967]; is a type of GO:0090227; positively regulates red or far-red light signaling pathway [GO:0010017]